{
  "term_id": "GO:0051015",
  "gene_name": "Alpha-actinin-2",
  "gene_symbol": "ACTN2",
  "term_label": "actin filament binding",
  "gene": "UniProtKB:P35609"
}